{
  "term_label": "nucleus",
  "gene_name": "Homeobox protein notochord",
  "term_id": "GO:0005634",
  "gene": "UniProtKB:A8MTQ0",
  "gene_symbol": "NOTO"
}